positive regulation of termination of RNA polymerase II transcription [GO:1904595] (biological process) References: PMID:25417108 Sources: GOC:TermGenie, GO_REF:0000058 Subtypes: GO:2000806 Definition: Any process that activates or increases the frequency, rate or extent of termination of RNA polymerase II transcription. Relationships: is a type of positive regulation of termination of DNA-templated transcription [GO:0060566]; is a type of regulation of termination of RNA polymerase II transcription [GO:1904594]; positively regulates termination of RNA polymerase II transcription [GO:0006369] Also known as: positive regulation of RNA 3'-end formation by RNA polymerase II, positive regulation of RNA polymerase II transcription termination, positive regulation of transcription termination from Pol II promoter, positive regulation of transcription termination from RNA polymerase II promoter, up regulation of RNA 3'-end formation by RNA polymerase II, up regulation of RNA polymerase II transcription termination, up regulation of termination of RNA polymerase II transcription, up regulation of transcription termination from Pol II promoter, up regulation of transcription termination from RNA polymerase II promoter, up-regulation of RNA 3'-end formation by RNA polymerase II, up-regulation of RNA polymerase II transcription termination, up-regulation of termination of RNA polymerase II transcription, up-regulation of transcription termination from Pol II promoter, up-regulation of transcription termination from RNA polymerase II promoter, upregulation of RNA 3'-end formation by RNA polymerase II, upregulation of RNA polymerase II transcription termination, upregulation of termination of RNA polymerase II transcription, upregulation of transcription termination from Pol II promoter, upregulation of transcription termination from RNA polymerase II promoter, activation of RNA 3'-end formation by RNA polymerase II, activation of RNA polymerase II transcription termination, activation of termination of RNA polymerase II transcription, activation of transcription termination from Pol II promoter, activation of transcription termination from RNA polymerase II promoter, activation of RNA polymerase II transcription termination factor activity, positive regulation of RNA polymerase II transcription termination factor activity, up regulation of RNA polymerase II transcription termination factor activity, up-regulation of RNA polymerase II transcription termination factor activity, upregulation of RNA polymerase II transcription termination factor activity